catechol-containing compound catabolic process [GO:0019614] (biological process) Sources: GOC:go_curators Also known as: catechol breakdown, catechol catabolic process, catechol catabolism, catechol degradation Relationships: is a type of GO:0009712; is a type of phenol-containing compound catabolic process [GO:0019336] Subtypes: catechol catabolic process, ortho-cleavage [GO:0019615], catechol catabolic process, meta-cleavage [GO:0019616], 3,4-dihydroxybenzoate catabolic process [GO:0019619], GO:0042424, chrysobactin catabolic process [GO:0042859], enterobactin catabolic process [GO:0046214], GO:0046276, GO:1900577, violaceol I catabolic process [GO:1900589], violaceol II catabolic process [GO:1900592], GO:1900798, 3-chlorocatechol catabolic process [GO:1901168], 3-(2,3-dihydroxyphenyl)propanoate catabolic process [GO:1901791] Definition: The chemical reactions and pathways resulting in the breakdown of catechol-containing compounds. Catechol is a compound containing a pyrocatechol nucleus or substituent.